{
  "gene_name": "Protein FAM180A",
  "term_id": "UNKNOWN:0002",
  "gene": "UniProtKB:Q6UWF9",
  "gene_symbol": "FAM180A",
  "term_label": "Unknown biological process"
}